{
  "gene_name": "UDP-glucuronic acid decarboxylase 1",
  "gene_symbol": "UXS1",
  "term_id": "GO:0070403",
  "term_label": "NAD+ binding",
  "gene": "UniProtKB:Q8NBZ7"
}